{
  "gene_name": "Zinc finger protein 322",
  "term_label": "Unknown cellular component",
  "term_id": "UNKNOWN:0003",
  "gene": "UniProtKB:Q6U7Q0",
  "gene_symbol": "ZNF322"
}